epinephrine secretion, neurotransmission [GO:0061529] (biological process) Relationships: is a type of epinephrine secretion [GO:0048242]; is a type of GO:0160043 Definition: The regulated release of epinephrine by a cell in which the epinephrine acts as a neurotransmitter. Sources: GOC:dph Also known as: adrenaline secretion, neurotransmission